{
  "gene_symbol": "PGA4",
  "gene": "UniProtKB:P0DJD7",
  "term_id": "GO:0004190",
  "term_label": "aspartic-type endopeptidase activity",
  "gene_name": "Pepsin A-4"
}